{
  "gene": "UniProtKB:P29762",
  "term_id": "GO:0005634",
  "gene_name": "Cellular retinoic acid-binding protein 1",
  "term_label": "nucleus",
  "gene_symbol": "CRABP1"
}